{
  "term_id": "UNKNOWN:0001",
  "term_label": "Unknown molecular function",
  "gene": "UniProtKB:P49746",
  "gene_name": "Thrombospondin-3",
  "gene_symbol": "THBS3"
}